{
  "gene": "UniProtKB:P04440",
  "gene_symbol": "HLA-DPB1",
  "term_label": "MHC class II protein complex",
  "term_id": "GO:0042613",
  "gene_name": "HLA class II histocompatibility antigen, DP beta 1 chain"
}